{
  "gene_name": "Armadillo repeat-containing protein 3",
  "term_label": "Unknown biological process",
  "gene_symbol": "ARMC3",
  "term_id": "UNKNOWN:0002",
  "gene": "UniProtKB:Q5W041"
}